protein O-linked glycosylation via arabinose [GO:0180063] (biological process) Also known as: protein O-linked arabinosylation References: PMID:33815452 Relationships: is a type of GO:0006493 Definition: A glycoprotein biosynthetic process starting with the covalent linkage of an arabinose via a beta-glycosidic bond to the oxygen atom of the hydroxyl group of a hydroxyproline in a protein, which can be further elongated with the sequential addition of sugar units resulting in the formation of a protein O-linked glycan.